{
  "term_id": "GO:0005634",
  "gene_name": "Zinc finger protein 530",
  "gene_symbol": "ZNF530",
  "term_label": "nucleus",
  "gene": "UniProtKB:Q6P9A1"
}